{
  "term_id": "GO:0016342",
  "gene": "UniProtKB:P55290",
  "term_label": "catenin complex",
  "gene_symbol": "CDH13",
  "gene_name": "Cadherin-13"
}